positive regulation of transporter activity [GO:0032411] (biological process) Sources: GOC:mah Also known as: up regulation of transporter activity, up-regulation of transporter activity, upregulation of transporter activity, activation of transporter activity, stimulation of transporter activity Relationships: is a type of positive regulation of molecular function [GO:0044093]; is a type of positive regulation of transport [GO:0051050]; positively regulates GO:0005215 Definition: Any process that activates or increases the activity of a transporter. Subtypes: GO:0032414, positive regulation of phospholipid scramblase activity [GO:1900163], positive regulation of oxidative phosphorylation uncoupler activity [GO:2000277]